{
  "gene_symbol": "WIPI1",
  "term_label": "phosphatidylinositol-3,5-bisphosphate binding",
  "gene": "UniProtKB:Q5MNZ9",
  "term_id": "GO:0080025",
  "gene_name": "WD repeat domain phosphoinositide-interacting protein 1"
}